{
  "term_label": "Golgi apparatus",
  "gene": "UniProtKB:Q6UWI2",
  "gene_symbol": "PARM1",
  "gene_name": "Prostate androgen-regulated mucin-like protein 1",
  "term_id": "GO:0005794"
}